{
  "gene_name": "Neuroblastoma breakpoint family member 1",
  "gene": "UniProtKB:Q3BBV0",
  "gene_symbol": "NBPF1",
  "term_id": "UNKNOWN:0001",
  "term_label": "Unknown molecular function"
}